{
  "gene_name": "Protein SETSIP",
  "gene": "UniProtKB:P0DME0",
  "term_id": "GO:0000785",
  "gene_symbol": "SETSIP",
  "term_label": "chromatin"
}